{
  "term_label": "estrogen metabolic process",
  "gene": "UniProtKB:Q9HAW8",
  "gene_symbol": "UGT1A10",
  "term_id": "GO:0008210",
  "gene_name": "UDP-glucuronosyltransferase 1A10"
}